{
  "term_id": "GO:0005829",
  "gene_symbol": "ZWINT",
  "gene": "UniProtKB:O95229",
  "gene_name": "ZW10 interactor",
  "term_label": "cytosol"
}